clathrin-sculpted glutamate transport vesicle lumen [GO:0060204] (cellular component) Definition: The volume enclosed by the membrane of the clathrin-sculpted glutamate transport vesicle. Sources: GOC:dph Also known as: clathrin sculpted glutamate constitutive secretory pathway transport vesicle lumen, clathrin sculpted glutamate transport vesicle lumen Relationships: is a type of cytoplasmic vesicle lumen [GO:0060205]; is part of clathrin-sculpted glutamate transport vesicle [GO:0060199]